{
  "term_label": "regulation of transcription by RNA polymerase II",
  "gene": "UniProtKB:Q9NZI6",
  "term_id": "GO:0006357",
  "gene_name": "Transcription factor CP2-like protein 1",
  "gene_symbol": "TFCP2L1"
}